{
  "gene_name": "Ubiquitin carboxyl-terminal hydrolase 28",
  "gene": "UniProtKB:Q96RU2",
  "term_id": "GO:0000077",
  "gene_symbol": "USP28",
  "term_label": "DNA damage checkpoint signaling"
}